{
  "gene_symbol": "CAPNS1",
  "gene_name": "Calpain small subunit 1",
  "term_id": "GO:0110158",
  "term_label": "calpain complex",
  "gene": "UniProtKB:P04632"
}